{
  "term_label": "ephrin receptor binding",
  "gene_name": "Cytoplasmic protein NCK1",
  "gene": "UniProtKB:P16333",
  "term_id": "GO:0046875",
  "gene_symbol": "NCK1"
}